positive regulation of cell proliferation involved in kidney development [GO:1901724] (biological process) Also known as: up regulation of cell proliferation involved in kidney development, up-regulation of cell proliferation involved in kidney development, upregulation of cell proliferation involved in kidney development, activation of cell proliferation involved in kidney development Relationships: is a type of positive regulation of cell population proliferation [GO:0008284]; is a type of regulation of cell proliferation involved in kidney development [GO:1901722]; positively regulates cell proliferation involved in kidney development [GO:0072111] Subtypes: positive regulation of glomerular mesangial cell proliferation [GO:0072126], GO:0090096, GO:2000608 Definition: Any process that activates or increases the frequency, rate or extent of cell proliferation involved in kidney development. References: PMID:18182616 Sources: GOC:TermGenie